{
  "gene_name": "Small ribosomal subunit protein uS3",
  "gene": "UniProtKB:P23396",
  "gene_symbol": "RPS3",
  "term_id": "GO:0005634",
  "term_label": "nucleus"
}